{
  "gene_symbol": "ADAM5",
  "gene": "UniProtKB:Q6NVV9",
  "term_id": "UNKNOWN:0001",
  "gene_name": "Putative disintegrin and metalloproteinase domain-containing protein 5",
  "term_label": "Unknown molecular function"
}